{
  "term_label": "odorant binding",
  "gene_symbol": "OR5B2",
  "gene_name": "Olfactory receptor 5B2",
  "term_id": "GO:0005549",
  "gene": "UniProtKB:Q96R09"
}